cellular detoxification of aldehyde [GO:0110095] (biological process) Relationships: is a type of GO:1990748; is part of GO:0110096 References: PMID:25656103 Sources: GOC:vw Definition: Any process carried out at the cellular level that reduces or removes the toxicity of an aldehyde. These may include transport of aldehydes away from sensitive areas and to compartments or complexes whose purpose is sequestration of the toxic substance. Subtypes: formaldehyde catabolic process [GO:0046294], cellular detoxification of methylglyoxal [GO:0140041]